mitotic division septum assembly [GO:0140278] (biological process) Definition: The assembly and arrangement of a septum that spans the plasma membrane interface between progeny cells following mitotic cytokinesis. The progeny cells that form a division septum are not able to exchange intracellular material. Regulation: regulated by regulation of mitotic division septum assembly [GO:0140279]; negatively regulated by negative regulation of mitotic division septum assembly [GO:0140280]; positively regulated by positive regulation of mitotic division septum assembly [GO:0140281] Relationships: is a type of GO:0000917; is a type of mitotic cytokinetic process [GO:1902410] References: PMID:22786806